{
  "gene": "UniProtKB:Q9BXJ5",
  "term_id": "UNKNOWN:0003",
  "gene_symbol": "C1QTNF2",
  "term_label": "Unknown cellular component",
  "gene_name": "Complement C1q tumor necrosis factor-related protein 2"
}